{
  "term_label": "Unknown cellular component",
  "gene_symbol": "GSDMA",
  "gene_name": "Gasdermin-A",
  "term_id": "UNKNOWN:0003",
  "gene": "UniProtKB:Q96QA5"
}